{
  "gene_name": "Neuropeptide W",
  "term_id": "GO:0001664",
  "gene": "UniProtKB:Q8N729",
  "gene_symbol": "NPW",
  "term_label": "G protein-coupled receptor binding"
}